{
  "term_label": "intracellular signal transduction",
  "gene_name": "Serine_threonine-protein kinase 24",
  "gene": "UniProtKB:Q9Y6E0",
  "gene_symbol": "STK24",
  "term_id": "GO:0035556"
}